neurotransmitter receptor regulator activity [GO:0099602] (molecular function) Definition: A molecular function that directly (via physical interaction or direct modification) activates, inhibits or otherwise modulates the activity of a neurotransmitter receptor. Modulation of activity includes changes in desensitization rate, ligand affinity, ion selectivity and pore-opening/closing. Relationships: is a type of GO:0030545; regulates neurotransmitter receptor activity [GO:0030594] References: PMID:12740117, PMID:18387948 Sources: GOC:dos Subtypes: GO:0030548